negative regulation of retinal cone cell fate commitment [GO:0060226] (biological process) Relationships: is a type of negative regulation of cell fate commitment [GO:0010454]; is a type of negative regulation of photoreceptor cell differentiation [GO:0046533]; is a type of regulation of retinal cone cell fate commitment [GO:0060222]; RO_0002212 retinal cone cell fate commitment [GO:0046551] Subtypes: negative regulation of retinal cone cell fate specification [GO:0009998] Sources: GOC:dph Definition: Any process that increases the process in which a cell becomes committed to a retinal cone cell fate. Retinal cone cell fate commitment is the process in which the developmental fate of a cell becomes restricted such that it will develop into a retinal cone cell.